regulation of cell proliferation involved in imaginal disc-derived wing morphogenesis [GO:0090256] (biological process) Relationships: is a type of regulation of cell population proliferation [GO:0042127]; is a type of regulation of post-embryonic development [GO:0048580]; is part of imaginal disc-derived wing morphogenesis [GO:0007476]; regulates GO:0090255 Sources: GOC:ascb_2009, GOC:dph, GOC:tb Definition: Any process that modulates the frequency, rate, or extent of the multiplication or reproduction of cells, resulting in the expansion of a cell population that contributes to imaginal disc-derived wing morphogenesis.